{
  "gene": "UniProtKB:Q8N4C8",
  "gene_name": "Misshapen-like kinase 1",
  "term_id": "GO:0043408",
  "gene_symbol": "MINK1",
  "term_label": "regulation of MAPK cascade"
}